{
  "gene_symbol": "DLGAP2",
  "gene_name": "Disks large-associated protein 2",
  "gene": "UniProtKB:Q9P1A6",
  "term_id": "GO:0099572",
  "term_label": "postsynaptic specialization"
}